{
  "gene_name": "Neuropilin-2",
  "term_id": "GO:0098978",
  "gene": "UniProtKB:O60462",
  "term_label": "glutamatergic synapse",
  "gene_symbol": "NRP2"
}